{
  "gene": "UniProtKB:P51606",
  "gene_name": "N-acylglucosamine 2-epimerase",
  "term_id": "GO:0050121",
  "gene_symbol": "RENBP",
  "term_label": "N-acylglucosamine 2-epimerase activity"
}